{
  "gene": "UniProtKB:Q2VIQ3",
  "term_id": "GO:0051231",
  "term_label": "spindle elongation",
  "gene_name": "Chromosome-associated kinesin KIF4B",
  "gene_symbol": "KIF4B"
}